U4atac/U6atac snRNP [GO:0071002] (cellular component) Definition: A ribonucleoprotein complex that contains the extensively base paired small nuclear RNAs U4atac and U6atac, a heptameric ring of Sm proteins associated with U4atac, the Lsm2-8 heptameric ring complex associated with U6atac, as well as several proteins that are unique to the U4atac snRNP or U6atac snRNPs, some of which remain associated with the U4atac/U6atac snRNA both while the U4atac snRNP is free or assembled into a series of spliceosomal complexes. References: PMID:14685174 Sources: GOC:krc, GOC:mah, ISBN:0879695897 Relationships: is a type of spliceosomal snRNP complex [GO:0097525]; BFO_0000051 GO:0005690; has part U6atac snRNP [GO:0005691]